{
  "gene": "UniProtKB:P21964",
  "term_label": "catechol O-methyltransferase activity",
  "gene_name": "Catechol O-methyltransferase",
  "term_id": "GO:0016206",
  "gene_symbol": "COMT"
}